{
  "term_label": "Unknown biological process",
  "gene_symbol": "ANKRD60",
  "gene": "UniProtKB:Q9BZ19",
  "term_id": "UNKNOWN:0002",
  "gene_name": "Ankyrin repeat domain-containing protein 60"
}